1,8-dihydroxynaphthalene-melanin biosynthetic process [GO:0140614] (biological process) Also known as: DHN-melanin biosynthesis Definition: The chemical reactions and pathways resulting in the formation of dihydroxy naphthalene (DHN)-melanin. Relationships: is a type of siderophore biosynthetic process [GO:0019290]; is_a GO:0030639; is a type of melanin biosynthetic process [GO:0042438] References: PMID:12788746, PMID:23998343